methyltetrahydroprotoberberine 14-monooxygenase activity [GO:0047084] (molecular function) Also known as: methyltetrahydroprotoberberine 14-hydroxylase activity, (S)-N-methylcanadine,NADPH:oxygen oxidoreductase (14-hydroxylating), (S)-cis-N-methyltetrahydroberberine 14-monooxygenase activity, (S)-cis-N-methyltetrahydroprotoberberine-14-hydroxylase activity Relationships: is a type of oxidoreductase activity, acting on paired donors, with incorporation or reduction of molecular oxygen, NAD(P)H as one donor, and incorporation of one atom of oxygen [GO:0016709] Sources: EC:1.14.14.97, MetaCyc:1.14.13.37-RXN Definition: Catalysis of the reaction: O2 + NADPH + H+ + (S)-N-methylcanadine = H2O + NADP+ + allocryptopine.